phloem sucrose loading [GO:0009915] (biological process) Definition: The process of loading sucrose into the sieve tube or companion cell of the phloem for long distance transport from source to sink. Relationships: is a type of GO:0015770; is a type of phloem loading [GO:0110126] Sources: GOC:sm